{
  "gene": "UniProtKB:C9JN71",
  "term_id": "GO:0006357",
  "gene_name": "Zinc finger protein 878",
  "gene_symbol": "ZNF878",
  "term_label": "regulation of transcription by RNA polymerase II"
}